{
  "gene_symbol": "SEMA4F",
  "gene_name": "Semaphorin-4F",
  "term_id": "GO:0005886",
  "term_label": "plasma membrane",
  "gene": "UniProtKB:O95754"
}